{
  "gene_symbol": "VEGFC",
  "term_id": "GO:0060754",
  "term_label": "positive regulation of mast cell chemotaxis",
  "gene_name": "Vascular endothelial growth factor C",
  "gene": "UniProtKB:P49767"
}